axon cytoplasm [GO:1904115] (cellular component) References: PMID:18667152 Sources: GOC:TermGenie, GO_REF:0000064 Relationships: is a type of neuron projection cytoplasm [GO:0120111]; is part of axon [GO:0030424] Also known as: axoplasm Definition: Any cytoplasm that is part of a axon.